{
  "gene": "UniProtKB:Q58FF7",
  "term_label": "protein stabilization",
  "gene_symbol": "HSP90AB3P",
  "term_id": "GO:0050821",
  "gene_name": "Putative heat shock protein HSP 90-beta-3"
}